{
  "gene_name": "Syntaxin-3",
  "term_id": "GO:0005886",
  "term_label": "plasma membrane",
  "gene": "UniProtKB:Q13277",
  "gene_symbol": "STX3"
}